{
  "term_id": "GO:0060070",
  "gene_name": "Frizzled-3",
  "gene": "UniProtKB:Q9NPG1",
  "term_label": "canonical Wnt signaling pathway",
  "gene_symbol": "FZD3"
}